{
  "gene": "UniProtKB:A0A0B4J2A2",
  "gene_symbol": "PPIAL4C",
  "term_label": "cyclosporin A binding",
  "gene_name": "Peptidyl-prolyl cis-trans isomerase A-like 4C",
  "term_id": "GO:0016018"
}